{
  "gene_symbol": "H2BC3",
  "gene_name": "Histone H2B type 1-B",
  "term_id": "GO:0005634",
  "gene": "UniProtKB:P33778",
  "term_label": "nucleus"
}